deoxyuridine 1'-dioxygenase activity [GO:0047079] (molecular function) Sources: EC:1.14.11.10, RHEA:23316 Also known as: pyrimidine-deoxynucleoside 1'-dioxygenase activity, pyrimidine-deoxynucleoside,2-oxoglutarate 1'-dioxygenase activity, 2'-deoxyuridine,2-oxoglutarate:oxygen oxidoreductase (1'-hydroxylating) Relationships: is a type of 2-oxoglutarate-dependent dioxygenase activity [GO:0016706] Definition: Catalysis of the reaction: 2'-deoxyuridine + 2-oxoglutarate + O2 = 2-deoxy-D-ribono-1,4-lactone + CO2 + succinate + uracil.